{
  "gene_symbol": "A0A1W2PQM1",
  "gene_name": "Immunoglobulin subtype domain-containing protein",
  "term_label": "Unknown biological process",
  "term_id": "UNKNOWN:0002",
  "gene": "UniProtKB:A0A1W2PQM1"
}